{
  "term_id": "GO:0000981",
  "gene_name": "Zinc finger protein 575",
  "gene": "UniProtKB:Q86XF7",
  "term_label": "DNA-binding transcription factor activity, RNA polymerase II-specific",
  "gene_symbol": "ZNF575"
}